{
  "gene": "UniProtKB:Q96NT0",
  "term_label": "Unknown cellular component",
  "gene_name": "Coiled-coil domain-containing protein 115",
  "term_id": "UNKNOWN:0003",
  "gene_symbol": "VMA22"
}